9+2 motile cilium [GO:0097729] (cellular component) Relationships: is_a GO:0031514; has part radial spoke [GO:0001534]; has part inner dynein arm [GO:0036156]; has part GO:0036157; has part axonemal central pair [GO:0097540]; has part axonemal doublet microtubule [GO:0097545] Note: This type of cilia may be present in solitary (so-called flagella, e.g. in sperm) or in multiple copies (so-called conventional motile cilia, e.g. in tracheal epithelium, ependyma or oviduct epithelium). Subtypes: GO:0036126, left anterior flagellum [GO:0097554], right anterior flagellum [GO:0097555], left posteriolateral flagellum [GO:0097556], right posteriolateral flagellum [GO:0097557], left ventral flagellum [GO:0097558], right ventral flagellum [GO:0097559], left caudal flagellum [GO:0097560], right caudal flagellum [GO:0097561], transverse flagellum [GO:0097608], longitudinal flagellum [GO:0097609] References: PMID:22118931 Sources: GOC:cilia Definition: A motile cilium where the axoneme has a ring of nine outer microtubule doublets plus two central microtubules (and is therefore called a 9+2 axoneme). Also known as: motile 9+2 cilium, conventional motile cilium, sperm flagellum